{
  "gene_symbol": "THEM4",
  "term_label": "mitochondrion",
  "term_id": "GO:0005739",
  "gene": "UniProtKB:Q5T1C6",
  "gene_name": "Acyl-coenzyme A thioesterase THEM4"
}